regulation of tubulin deacetylation [GO:0090043] (biological process) Definition: Any process that modulates the frequency, rate or extent of tubulin deacetylation. Tubulin deacetylation is the removal of an acetyl group from a protein amino acid. Sources: GOC:BHF, GOC:dph, GOC:tb Relationships: is a type of regulation of protein deacetylation [GO:0090311]; regulates GO:0090042 Subtypes: positive regulation of tubulin deacetylation [GO:0090044], negative regulation of tubulin deacetylation [GO:1904428]